{
  "gene_symbol": "TXNRD2",
  "gene_name": "Thioredoxin reductase 2, mitochondrial",
  "gene": "UniProtKB:Q9NNW7",
  "term_label": "cytoplasm",
  "term_id": "GO:0005737"
}